{
  "term_label": "reduction of food intake in response to dietary excess",
  "gene_name": "Growth_differentiation factor 15",
  "term_id": "GO:0002023",
  "gene_symbol": "GDF15",
  "gene": "UniProtKB:Q99988"
}